histone H3K9 trimethyltransferase activity [GO:0140949] (molecular function) Relationships: is a type of histone H3K9 methyltransferase activity [GO:0046974] Definition: Catalysis of the reaction: L-lysyl9-[histone H3] + 3 S-adenosyl-L-methionine = 3 H+ + N6,N6,N6-trimethyl-L-lysyl9-[histone H3] + 3 S-adenosyl-L-homocysteine. This reaction is the successive addition of three methyl groups to the unmethylated lysine residue at position 9 of histone H3, producing histone H3K9me3. Also known as: histone H3-K9 trimethylation, histone H3K9 trimethylation, histone H3K9 mono/di/trimethylase activity, histone H3K9 trimethylase activity, histone lysine N-trimethyltransferase activity (H3-K9 specific) Note: Comment: Note that the residue position corresponds to the canonical human H3 histone (UniProtKB:P84243); this residue is conserved across all eukaryotes. Residue 1 is the first residue following removal of the initiating Methionine (Met). Note that each histone is encoded by multiple genes, and sequences may vary across different genes within an organism. Sources: RHEA:60276